DNA ligase IV complex [GO:0032807] (cellular component) References: PMID:16314503 Definition: A eukaryotically conserved protein complex that contains DNA ligase IV and is involved in DNA repair by non-homologous end joining; in addition to the ligase, the complex also contains XRCC4 or a homolog, e.g. Saccharomyces Lif1p. Relationships: is a type of nonhomologous end joining complex [GO:0070419]; is a type of GO:0140513 Also known as: DNA ligase IV-XRCC4 complex